{
  "gene": "UniProtKB:Q92526",
  "term_id": "GO:0051082",
  "gene_name": "T-complex protein 1 subunit zeta-2",
  "term_label": "unfolded protein binding",
  "gene_symbol": "CCT6B"
}